{
  "gene_name": "U6 snRNA-associated Sm-like protein LSm4",
  "term_label": "P-body assembly",
  "gene": "UniProtKB:Q9Y4Z0",
  "term_id": "GO:0033962",
  "gene_symbol": "LSM4"
}